{
  "gene": "UniProtKB:Q8IZX4",
  "gene_symbol": "TAF1L",
  "term_label": "transcription factor TFIID complex",
  "term_id": "GO:0005669",
  "gene_name": "Transcription initiation factor TFIID subunit 1-like"
}